{
  "term_id": "UNKNOWN:0002",
  "term_label": "Unknown biological process",
  "gene_name": "Fibroblast growth factor receptor-like 1",
  "gene": "UniProtKB:Q8N441",
  "gene_symbol": "FGFRL1"
}